negative regulation of Lewy body formation [GO:0140123] (biological process) Sources: GOC:sl Relationships: is a type of negative regulation of inclusion body assembly [GO:0090084]; is a type of regulation of Lewy body formation [GO:0140122]; negatively regulates GO:0140121 Definition: Any process that stops, prevents or reduces the frequency, rate or extent of Lewy body formation.